{
  "term_label": "epsilon DNA polymerase complex",
  "term_id": "GO:0008622",
  "gene_symbol": "POLE3",
  "gene_name": "DNA polymerase epsilon subunit 3",
  "gene": "UniProtKB:Q9NRF9"
}